cellular response to hydrogen peroxide [GO:0070301] (biological process) Sources: CHEBI:16240, GOC:mah Relationships: is a type of GO:0034614; is a type of response to hydrogen peroxide [GO:0042542] Definition: Any process that results in a change in state or activity of a cell (in terms of movement, secretion, enzyme production, gene expression, etc.) as a result of a hydrogen peroxide (H2O2) stimulus.